{
  "term_id": "GO:0005886",
  "gene_name": "Zinc transporter ZIP1",
  "gene": "UniProtKB:Q9NY26",
  "gene_symbol": "SLC39A1",
  "term_label": "plasma membrane"
}